{
  "gene_symbol": "AR",
  "gene": "UniProtKB:P10275",
  "gene_name": "Androgen receptor",
  "term_label": "estrogen response element binding",
  "term_id": "GO:0034056"
}